sulfur oxidation [GO:0019417] (biological process) Definition: The chemical reactions and pathways resulting the addition of oxygen to elemental sulfur. Also known as: sulphur oxidation Sources: GOC:jl Relationships: is a type of sulfur compound metabolic process [GO:0006790] Subtypes: sulfur oxidation, ferric ion-dependent [GO:0019423], aerobic sulfur oxidation [GO:0070220]